{
  "term_id": "GO:0048384",
  "term_label": "retinoic acid receptor signaling pathway",
  "gene_symbol": "RARA",
  "gene": "UniProtKB:P10276",
  "gene_name": "Retinoic acid receptor alpha"
}